{
  "gene_symbol": "TLR8",
  "gene_name": "Toll-like receptor 8",
  "gene": "UniProtKB:Q9NR97",
  "term_label": "canonical NF-kappaB signal transduction",
  "term_id": "GO:0007249"
}